{
  "gene_name": "Non-receptor tyrosine-protein kinase TNK1",
  "term_label": "protein tyrosine kinase activity",
  "term_id": "GO:0004713",
  "gene": "UniProtKB:Q13470",
  "gene_symbol": "TNK1"
}